{
  "term_label": "endosome organization",
  "gene": "UniProtKB:Q9H270",
  "gene_name": "Vacuolar protein sorting-associated protein 11 homolog",
  "gene_symbol": "VPS11",
  "term_id": "GO:0007032"
}